leaf papilla [GO:0090396] (cellular component) Note: Part of leaf papilla cell (PO:0025167). Sources: GOC:tb Relationships: is a type of plant cell papilla [GO:0090395] Definition: A plant cell papilla that is part of a leaf papilla cell.